negative regulation of dephosphorylation [GO:0035305] (BP) Subtypes: negative regulation of phosphatase activity [GO:0010923] Sources: GOC:bf Definition: Any process the stops, prevents, or reduces the frequency, rate or extent of removal of phosphate groups from a molecule. Also known as: down regulation of dephosphorylation, down-regulation of dephosphorylation, downregulation of dephosphorylation, inhibition of dephosphorylation Relationships: is a type of regulation of dephosphorylation [GO:0035303]; is a type of GO:0045936; negatively regulates dephosphorylation [GO:0016311]